{
  "gene": "UniProtKB:P19957",
  "term_id": "GO:0005615",
  "term_label": "extracellular space",
  "gene_name": "Elafin",
  "gene_symbol": "PI3"
}